negative regulation of cellular respiration [GO:1901856] (biological process) References: PMID:23150719 Sources: GOC:TermGenie, GOC:yaf Definition: Any process that stops, prevents or reduces the frequency, rate or extent of cellular respiration. Relationships: is_a negative regulation of metabolic process [GO:0009892]; is a type of regulation of cellular respiration [GO:0043457]; negatively regulates GO:0045333 Also known as: down regulation of respiration, down-regulation of respiration, downregulation of respiration, inhibition of respiration, negative regulation of respiration, down regulation of cellular respiration, down regulation of oxidative metabolic process, down regulation of oxidative metabolism, down-regulation of cellular respiration, down-regulation of oxidative metabolic process, down-regulation of oxidative metabolism, downregulation of cellular respiration, downregulation of oxidative metabolic process, downregulation of oxidative metabolism, inhibition of oxidative metabolic process, inhibition of oxidative metabolism, negative regulation of oxidative metabolic process, negative regulation of oxidative metabolism, inhibition of cellular respiration Subtypes: negative regulation of oxidative phosphorylation [GO:0090324], negative regulation of methane biosynthetic process from dimethylamine [GO:1900319], GO:1900331, GO:1900334, negative regulation of methane biosynthetic process from carbon monoxide [GO:1900337], negative regulation of methane biosynthetic process from formic acid [GO:1900340], negative regulation of methane biosynthetic process from dimethyl sulfide [GO:1900343], negative regulation of methane biosynthetic process from methanethiol [GO:1900346], negative regulation of methane biosynthetic process from methylamine [GO:1900349]